{
  "term_id": "GO:0008631",
  "gene_name": "Diablo IAP-binding mitochondrial protein",
  "gene": "UniProtKB:Q9NR28",
  "gene_symbol": "DIABLO",
  "term_label": "intrinsic apoptotic signaling pathway in response to oxidative stress"
}